{
  "term_label": "DNA translocase activity",
  "gene": "UniProtKB:Q2NKX8",
  "gene_name": "DNA excision repair protein ERCC-6-like",
  "term_id": "GO:0015616",
  "gene_symbol": "ERCC6L"
}